{
  "term_label": "Unknown molecular function",
  "gene_symbol": "ERVK-5",
  "gene_name": "Endogenous retrovirus group K member 5 Gag polyprotein",
  "gene": "UniProtKB:Q9HDB9",
  "term_id": "UNKNOWN:0001"
}